{
  "gene_name": "Beta-galactosidase-1-like protein 2",
  "term_id": "GO:0019388",
  "gene": "UniProtKB:Q8IW92",
  "gene_symbol": "GLB1L2",
  "term_label": "galactose catabolic process"
}